{
  "gene_name": "Interferon gamma",
  "term_id": "GO:0006959",
  "term_label": "humoral immune response",
  "gene": "UniProtKB:P01579",
  "gene_symbol": "IFNG"
}